{
  "gene": "UniProtKB:Q2V2M9",
  "term_id": "GO:0051015",
  "gene_name": "FH1_FH2 domain-containing protein 3",
  "gene_symbol": "FHOD3",
  "term_label": "actin filament binding"
}